{
  "term_id": "GO:0005737",
  "gene_symbol": "UBR1",
  "gene": "UniProtKB:Q8IWV7",
  "gene_name": "E3 ubiquitin-protein ligase UBR1",
  "term_label": "cytoplasm"
}